{
  "gene_name": "Zinc phosphodiesterase ELAC protein 2",
  "gene_symbol": "ELAC2",
  "term_id": "GO:1990180",
  "gene": "UniProtKB:Q9BQ52",
  "term_label": "mitochondrial tRNA 3'-end processing"
}